{
  "gene": "UniProtKB:Q86XE3",
  "term_id": "GO:1990246",
  "gene_symbol": "MICU3",
  "gene_name": "Calcium uptake protein 3, mitochondrial",
  "term_label": "uniplex complex"
}